{
  "gene_name": "TLC domain-containing protein 2",
  "term_label": "plasma membrane",
  "gene_symbol": "TLCD2",
  "term_id": "GO:0005886",
  "gene": "UniProtKB:A6NGC4"
}